{
  "term_id": "UNKNOWN:0001",
  "gene_name": "Uncharacterized protein encoded by LINC01600",
  "gene_symbol": "LINC01600",
  "gene": "UniProtKB:Q96MT4",
  "term_label": "Unknown molecular function"
}